{
  "gene": "UniProtKB:Q9P2D7",
  "gene_symbol": "DNAH1",
  "term_label": "dynein complex",
  "gene_name": "Dynein axonemal heavy chain 1",
  "term_id": "GO:0030286"
}